{
  "term_label": "Unknown biological process",
  "gene_symbol": "MATR3",
  "gene_name": "Matrin-3",
  "gene": "UniProtKB:P43243",
  "term_id": "UNKNOWN:0002"
}